{
  "gene_name": "Glutaminyl-peptide cyclotransferase-like protein",
  "gene": "UniProtKB:Q9NXS2",
  "term_id": "GO:0016603",
  "term_label": "glutaminyl-peptide cyclotransferase activity",
  "gene_symbol": "QPCTL"
}